{
  "gene_symbol": "HMGA1",
  "gene": "UniProtKB:P17096",
  "term_id": "GO:0005634",
  "gene_name": "High mobility group protein HMG-I_HMG-Y",
  "term_label": "nucleus"
}